{
  "gene_name": "ATP-binding cassette sub-family D member 2",
  "gene_symbol": "ABCD2",
  "term_label": "ATP binding",
  "gene": "UniProtKB:Q9UBJ2",
  "term_id": "GO:0005524"
}